{
  "gene_symbol": "DLX3",
  "term_id": "GO:0000978",
  "term_label": "RNA polymerase II cis-regulatory region sequence-specific DNA binding",
  "gene": "UniProtKB:O60479",
  "gene_name": "Homeobox protein DLX-3"
}